{
  "gene_name": "Membrane-associated tyrosine- and threonine-specific cdc2-inhibitory kinase",
  "term_id": "GO:0110031",
  "term_label": "negative regulation of G2/MI transition of meiotic cell cycle",
  "gene": "UniProtKB:Q99640",
  "gene_symbol": "PKMYT1"
}